cell-cell signaling involved in cell fate commitment [GO:0045168] (biological process) Definition: Signaling at long or short range between cells that results in the commitment of a cell to a certain fate. Sources: GOC:dph, GOC:go_curators, GOC:tb Relationships: is a type of cell-cell signaling [GO:0007267]; is part of cell fate commitment [GO:0045165] Also known as: cell fate commitment, cell-cell signaling, cell fate commitment, cell-cell signalling, cell-cell signaling during in cell fate commitment, cell-cell signaling resulting in cell fate commitment, cell-cell signalling during cell fate commitment, cell-cell signalling resulting in cell fate commitment, cell-cell signalling involved in cell fate specification Subtypes: lateral inhibition [GO:0046331], trichome patterning [GO:0048629]